{
  "term_id": "GO:0043065",
  "gene_name": "Bcl-2-modifying factor",
  "gene_symbol": "BMF",
  "term_label": "positive regulation of apoptotic process",
  "gene": "UniProtKB:Q96LC9"
}